{
  "gene": "UniProtKB:Q96KA5",
  "gene_symbol": "CLPTM1L",
  "term_id": "UNKNOWN:0002",
  "term_label": "Unknown biological process",
  "gene_name": "Lipid scramblase CLPTM1L"
}